UUU codon-amino acid adaptor activity [GO:0033401] (molecular function) Relationships: is a type of GO:0030533 Definition: A triplet codon-amino acid adaptor activity that recognizes a UUU codon. Sources: GOC:mah Also known as: TTT codon-amino acid adaptor activity, phenylalanine tRNA Note: Note that in the standard genetic code, TTT codes for phenylalanine.